specification of animal organ identity [GO:0010092] (biological process) Definition: The regionalization process in which the identity of an animal organ primordium is specified. Identity is considered to be the aggregate of characteristics by which a structure is recognized. Sources: GOC:tb Regulation: positively regulated by organ induction [GO:0001759] Relationships: is a type of GO:0003002; is part of animal organ formation [GO:0048645] Subtypes: heart field specification [GO:0003128], lung field specification [GO:0060424], prostate field specification [GO:0060515], GO:0060594, pancreas field specification [GO:0061131], kidney field specification [GO:0072004]